positive regulation of aspartic-type peptidase activity [GO:1905247] (biological process) Also known as: up regulation of aspartic-type peptidase activity, up-regulation of aspartic-type peptidase activity, upregulation of aspartic-type peptidase activity, activation of aspartic-type peptidase activity References: PMID:21745575 Sources: GOC:TermGenie, GOC:jl, GO_REF:0000059 Definition: Any process that activates or increases the frequency, rate or extent of aspartic-type peptidase activity. Relationships: is a type of positive regulation of peptidase activity [GO:0010952]; positively regulates aspartic-type peptidase activity [GO:0070001]